{
  "gene_symbol": "SEMA4G",
  "gene": "UniProtKB:Q9NTN9",
  "term_label": "positive regulation of cell migration",
  "term_id": "GO:0030335",
  "gene_name": "Semaphorin-4G"
}